organelle membrane fusion [GO:0090174] (biological process) Relationships: is a type of organelle fusion [GO:0048284]; is a type of membrane fusion [GO:0061025] Sources: GOC:ascb_2009, GOC:dph, GOC:tb Subtypes: GO:0000740, vesicle fusion [GO:0006906], GO:0016320, GO:0036504, karyomere membrane fusion [GO:0061472] Definition: The joining of two lipid bilayers to form a single organelle membrane.